{
  "term_id": "GO:0004984",
  "gene_symbol": "OR1K1",
  "term_label": "olfactory receptor activity",
  "gene_name": "Olfactory receptor 1K1",
  "gene": "UniProtKB:Q8NGR3"
}